{
  "gene_symbol": "SGK2",
  "term_label": "protein serine/threonine kinase activity",
  "gene": "UniProtKB:Q9HBY8",
  "gene_name": "Serine_threonine-protein kinase Sgk2",
  "term_id": "GO:0004674"
}